{
  "gene_name": "Leucine-rich repeat-containing protein 34",
  "gene_symbol": "LRRC34",
  "gene": "UniProtKB:Q8IZ02",
  "term_label": "Unknown molecular function",
  "term_id": "UNKNOWN:0001"
}